{
  "gene_symbol": "HSD3B2",
  "term_id": "GO:0016616",
  "gene_name": "3 beta-hydroxysteroid dehydrogenase_Delta 5--4-isomerase type 2",
  "term_label": "oxidoreductase activity, acting on the CH-OH group of donors, NAD or NADP as acceptor",
  "gene": "UniProtKB:P26439"
}